{
  "gene_name": "Cytidine deaminase",
  "term_label": "zinc ion binding",
  "term_id": "GO:0008270",
  "gene": "UniProtKB:P32320",
  "gene_symbol": "CDA"
}